acyl-CoA biosynthetic process [GO:0071616] (BP) Subtypes: GO:0006085, L-methylmalonyl-CoA biosynthetic process [GO:0019680], fatty-acyl-CoA biosynthetic process [GO:0046949], GO:1901290, benzoyl-CoA biosynthetic process [GO:1901789], 2-hydroxybenzoyl-CoA biosynthetic process [GO:1901887], malonyl-CoA biosynthetic process [GO:2001295] Regulation: regulated by regulation of acyl-CoA biosynthetic process [GO:0050812] Also known as: acyl-CoA anabolism, acyl-CoA biosynthesis, acyl-CoA formation, acyl-CoA synthesis Definition: The chemical reactions and pathways resulting in the formation of acyl-CoA, any derivative of coenzyme A in which the sulfhydryl group is in thiolester linkage with an acyl group. Relationships: is a type of acyl-CoA metabolic process [GO:0006637]; is a type of amide biosynthetic process [GO:0043604]; is a type of sulfur compound biosynthetic process [GO:0044272]; is a type of purine-containing compound biosynthetic process [GO:0072522]; is a type of nucleoside phosphate biosynthetic process [GO:1901293] Sources: GOC:cjk